{
  "term_label": "structural constituent of muscle",
  "gene_name": "Myosin light polypeptide 6",
  "gene_symbol": "MYL6",
  "gene": "UniProtKB:P60660",
  "term_id": "GO:0008307"
}